{
  "term_label": "Unknown biological process",
  "term_id": "UNKNOWN:0002",
  "gene": "UniProtKB:Q6ZMU1",
  "gene_symbol": "C3P1",
  "gene_name": "Putative protein C3P1"
}